membrane docking [GO:0022406] (biological process) References: PMID:27875684 Sources: GOC:isa_complete Relationships: is a type of cellular process [GO:0009987] Definition: The initial attachment of a membrane or protein to a target membrane. Docking requires only that the proteins come close enough to interact and adhere. Subtypes: membrane to membrane docking [GO:0022614], GO:0022615, GO:0140056